{
  "term_id": "GO:0045211",
  "gene_symbol": "KCNC2",
  "gene_name": "Potassium voltage-gated channel subfamily C member 2",
  "term_label": "postsynaptic membrane",
  "gene": "UniProtKB:Q96PR1"
}